{
  "gene_name": "Uncharacterized protein C17orf98",
  "term_id": "UNKNOWN:0003",
  "term_label": "Unknown cellular component",
  "gene_symbol": "C17orf98",
  "gene": "UniProtKB:A8MV24"
}